{
  "gene_symbol": "TEKT4",
  "gene": "UniProtKB:Q8WW24",
  "term_id": "GO:0015630",
  "term_label": "microtubule cytoskeleton",
  "gene_name": "Tektin-4"
}